{
  "gene": "UniProtKB:P61586",
  "gene_symbol": "RHOA",
  "gene_name": "Transforming protein RhoA",
  "term_label": "dendritic spine",
  "term_id": "GO:0043197"
}